{
  "term_label": "monoatomic anion transmembrane transport",
  "gene_symbol": "LRRC8C",
  "gene": "UniProtKB:Q8TDW0",
  "term_id": "GO:0098656",
  "gene_name": "Volume-regulated anion channel subunit LRRC8C"
}